{
  "term_id": "GO:0005739",
  "gene_symbol": "NMNAT3",
  "gene": "UniProtKB:Q96T66",
  "gene_name": "Nicotinamide_nicotinic acid mononucleotide adenylyltransferase 3",
  "term_label": "mitochondrion"
}